beta-N-acetylhexosaminidase complex [GO:1905379] (cellular component) References: PMID:6458607 Sources: GOC:TermGenie, GOC:bhm, GO_REF:0000088 Relationships: is a type of GO:1902494 Note: An example of this is HEXB in human (UniProt symbol P07686) in PMID:6458607 (inferred from direct assay). Also known as: HEX A complex, HEX B complex, HEX S complex Definition: A protein complex which is capable of beta-N-acetylhexosaminidase activity.